{
  "term_id": "GO:0043123",
  "gene_symbol": "IRAK1",
  "gene_name": "Interleukin-1 receptor-associated kinase 1",
  "gene": "UniProtKB:P51617",
  "term_label": "positive regulation of canonical NF-kappaB signal transduction"
}